{
  "gene_name": "Uncharacterized protein C5orf67",
  "term_label": "Unknown biological process",
  "gene_symbol": "C5orf67",
  "term_id": "UNKNOWN:0002",
  "gene": "UniProtKB:F2Z3F1"
}